{
  "gene_name": "BRCA1-associated protein",
  "gene_symbol": "BRAP",
  "term_id": "GO:0007265",
  "gene": "UniProtKB:Q7Z569",
  "term_label": "Ras protein signal transduction"
}